symbiont-containing vacuole membrane [GO:0020005] (cellular component) Relationships: is a type of GO:0031090; BFO_0000050 symbiont-containing vacuole [GO:0020003] Also known as: parasitophorous vacuolar membrane Definition: The lipid bilayer surrounding a symbiont-containing vacuole, derived from both the host and symbiont. Sources: GOC:jl, GOC:mb